{
  "term_id": "UNKNOWN:0002",
  "gene": "UniProtKB:Q5T230",
  "term_label": "Unknown biological process",
  "gene_symbol": "UTF1",
  "gene_name": "Undifferentiated embryonic cell transcription factor 1"
}